{
  "gene": "UniProtKB:Q9H3S1",
  "gene_symbol": "SEMA4A",
  "term_id": "GO:0038191",
  "term_label": "neuropilin binding",
  "gene_name": "Semaphorin-4A"
}